{
  "term_label": "attachment of spindle microtubules to kinetochore",
  "gene": "UniProtKB:Q6UWZ7",
  "gene_symbol": "ABRAXAS1",
  "gene_name": "BRCA1-A complex subunit Abraxas 1",
  "term_id": "GO:0008608"
}